{
  "gene_name": "Phospholipid-transporting ATPase IG",
  "term_label": "ATPase-coupled intramembrane lipid transporter activity",
  "gene": "UniProtKB:Q8NB49",
  "gene_symbol": "ATP11C",
  "term_id": "GO:0140326"
}